tRNA N2-guanine methylation [GO:0002940] (biological process) Sources: ISBN:155581073X, ISBN:1555811337 Also known as: tRNA m2-guanine biosynthesis Relationships: is a type of tRNA methylation [GO:0030488] Definition: The process whereby a guanine in a tRNA is methylated at the N2 position of guanine.